{
  "term_id": "GO:0005543",
  "gene_symbol": "CLINT1",
  "gene": "UniProtKB:Q14677",
  "gene_name": "Clathrin interactor 1",
  "term_label": "phospholipid binding"
}